{
  "gene_name": "Signal peptide, CUB and EGF-like domain-containing protein 2",
  "term_id": "GO:0005615",
  "gene_symbol": "SCUBE2",
  "gene": "UniProtKB:Q9NQ36",
  "term_label": "extracellular space"
}